{
  "gene": "UniProtKB:A6NGE7",
  "term_id": "UNKNOWN:0003",
  "gene_name": "Putative 2-oxo-4-hydroxy-4-carboxy-5-ureidoimidazoline decarboxylase",
  "term_label": "Unknown cellular component",
  "gene_symbol": "URAD"
}